cyanelle inner membrane [GO:0036012] (cellular component) Relationships: is_a plastid inner membrane [GO:0009528]; is a type of cyanelle membrane [GO:0033113] Definition: The inner, i.e. lumen-facing, lipid bilayer of the cyanelle envelope; also faces the cyanelle stroma. Also known as: cyanelle inner envelope membrane References: PMID:18976493 Sources: GOC:aa